{
  "term_label": "extracellular space",
  "gene_name": "Macrophage migration inhibitory factor",
  "term_id": "GO:0005615",
  "gene": "UniProtKB:P14174",
  "gene_symbol": "MIF"
}